BLOC-2 complex [GO:0031084] (cellular component) Relationships: is a type of BLOC complex [GO:0031082] Definition: A protein complex required for the biogenesis of specialized organelles of the endosomal-lysosomal system, such as melanosomes and platelet dense granules. The human complex contains the Hps3, Hps5, and Hps6 proteins; the mouse complex contains ru2 and ru. References: PMID:12548288, PMID:14718540, PMID:15031569